positive regulation of o-orsellinic acid biosynthetic process [GO:1900700] (biological process) Also known as: activation of o-orsellinic acid anabolism, activation of o-orsellinic acid biosynthesis, activation of o-orsellinic acid formation, activation of o-orsellinic acid synthesis, positive regulation of o-orsellinic acid anabolism, positive regulation of o-orsellinic acid biosynthesis, positive regulation of o-orsellinic acid formation, positive regulation of o-orsellinic acid synthesis, up regulation of o-orsellinic acid anabolism, up regulation of o-orsellinic acid biosynthesis, up regulation of o-orsellinic acid biosynthetic process, up regulation of o-orsellinic acid formation, up regulation of o-orsellinic acid synthesis, up-regulation of o-orsellinic acid anabolism, up-regulation of o-orsellinic acid biosynthesis, up-regulation of o-orsellinic acid biosynthetic process, up-regulation of o-orsellinic acid formation, up-regulation of o-orsellinic acid synthesis, upregulation of o-orsellinic acid anabolism, upregulation of o-orsellinic acid biosynthesis, upregulation of o-orsellinic acid biosynthetic process, upregulation of o-orsellinic acid formation, upregulation of o-orsellinic acid synthesis, activation of o-orsellinic acid biosynthetic process Definition: Any process that activates or increases the frequency, rate or extent of o-orsellinic acid biosynthetic process. Relationships: is a type of positive regulation of small molecule metabolic process [GO:0062013]; is a type of GO:1900378; is a type of GO:1900698; positively regulates GO:1900584 Sources: GOC:TermGenie, GOC:di